{
  "gene_name": "AP-3 complex subunit sigma-1",
  "gene_symbol": "AP3S1",
  "gene": "UniProtKB:Q92572",
  "term_label": "Unknown cellular component",
  "term_id": "UNKNOWN:0003"
}